{
  "gene": "UniProtKB:O94972",
  "term_label": "aggresome assembly",
  "term_id": "GO:0070842",
  "gene_name": "E3 ubiquitin-protein ligase TRIM37",
  "gene_symbol": "TRIM37"
}